{
  "term_label": "Unknown biological process",
  "gene_symbol": "FAM104A",
  "gene": "UniProtKB:Q969W3",
  "term_id": "UNKNOWN:0002",
  "gene_name": "Protein FAM104A"
}